negative regulation of entry into reproductive diapause [GO:0061964] (biological process) References: PMID:27689881 Sources: GOC:ha Definition: Any process that stops, prevents, or reduces the frequency, rate or extent of the dormancy process that results in entry into reproductive diapause. Reproductive diapause is a form of diapause where the organism itself will remain fully active, including feeding and other routine activities, but the reproductive organs experience a tissue-specific reduction in metabolism, with characteristic triggering and releasing stimuli. Relationships: is a type of negative regulation of developmental process [GO:0051093]; is a type of regulation of entry into reproductive diapause [GO:0061963]; negatively regulates entry into reproductive diapause [GO:0055116]